{
  "gene_name": "Immunoglobulin kappa variable 1-16",
  "term_label": "Unknown molecular function",
  "gene": "UniProtKB:P04430",
  "term_id": "UNKNOWN:0001",
  "gene_symbol": "IGKV1-16"
}